dendritic transport of messenger ribonucleoprotein complex [GO:0098963] (biological process) Relationships: is a type of dendritic transport [GO:0098935] Definition: The directed movement of a messenger ribonucleoprotein complex along microtubules in nerve cell dendrites. Also known as: dendritic transport of mRNA RNP complex Sources: GOC:dos